chromosome passenger complex localization to spindle midzone [GO:0035853] (biological process) Definition: A cellular protein complex localization that acts on a chromosome passenger complex; as a result, the complex is transported to, or maintained in, a specific location at the spindle midzone. A chromosome passenger complex is a protein complex that contains the BIR-domain-containing protein Survivin, Aurora B kinase, INCENP and Borealin, and coordinates various events based on its location to different structures during the course of mitosis. The spindle midzone is the area in the center of the spindle where the spindle microtubules from opposite poles overlap. References: PMID:15296749 Sources: GOC:mah, GOC:vw Also known as: CPC complex localization to spindle midzone, CPC localization to spindle midzone, chromosomal passenger complex localization to spindle midzone, chromosome passenger complex localisation to spindle midzone, chromosome passenger complex localization to central spindle, chromosome passenger complex localization to spindle equator Relationships: is a type of GO:0031503; is a type of protein localization to cytoskeleton [GO:0044380]